{
  "term_label": "neuropilin binding",
  "gene_symbol": "SEMA3C",
  "gene_name": "Semaphorin-3C",
  "gene": "UniProtKB:Q99985",
  "term_id": "GO:0038191"
}